{
  "gene_name": "Putative adrenomedullin-5-like protein",
  "gene": "UniProtKB:C9JUS6",
  "gene_symbol": "ADM5",
  "term_id": "GO:0005615",
  "term_label": "extracellular space"
}